{
  "gene": "UniProtKB:Q6ZVQ6",
  "gene_symbol": "Q6ZVQ6",
  "term_label": "Unknown biological process",
  "gene_name": "Putative uncharacterized protein FLJ42213",
  "term_id": "UNKNOWN:0002"
}